lamellipodium morphogenesis [GO:0072673] (BP) Definition: A process that is carried out at the cellular level and in which the structure of a lamellipodium is organized. Sources: GOC:BHF, GOC:mah Also known as: lamellipodium organization Relationships: is a type of lamellipodium organization [GO:0097581]; is a type of plasma membrane bounded cell projection morphogenesis [GO:0120039] Regulation: regulated by GO:2000392; negatively regulated by negative regulation of lamellipodium morphogenesis [GO:2000393]; positively regulated by positive regulation of lamellipodium morphogenesis [GO:2000394]